{
  "gene": "UniProtKB:Q7Z2H8",
  "term_label": "amino acid:proton symporter activity",
  "term_id": "GO:0005280",
  "gene_name": "Proton-coupled amino acid transporter 1",
  "gene_symbol": "SLC36A1"
}